{
  "gene": "UniProtKB:O43812",
  "term_label": "RNA polymerase II transcription regulatory region sequence-specific DNA binding",
  "gene_symbol": "DUX1",
  "gene_name": "Double homeobox protein 1",
  "term_id": "GO:0000977"
}